{
  "gene_symbol": "PIK3CG",
  "gene_name": "Phosphatidylinositol 4,5-bisphosphate 3-kinase catalytic subunit gamma isoform",
  "gene": "UniProtKB:P48736",
  "term_id": "GO:0016477",
  "term_label": "cell migration"
}